regulation of response to cytokine stimulus [GO:0060759] (biological process) Relationships: is_a regulation of response to stimulus [GO:0048583]; regulates GO:0034097 Sources: GOC:BHF, GOC:dph, GOC:tb Subtypes: regulation of cytokine-mediated signaling pathway [GO:0001959], GO:0060330, positive regulation of response to cytokine stimulus [GO:0060760], negative regulation of response to cytokine stimulus [GO:0060761], regulation of response to macrophage colony-stimulating factor [GO:1903969] Definition: Any process that modulates the rate, frequency, or extent of a response to cytokine stimulus.